{
  "gene_symbol": "ZBP1",
  "term_id": "GO:0060545",
  "gene_name": "Z-DNA-binding protein 1",
  "term_label": "positive regulation of necroptotic process",
  "gene": "UniProtKB:Q9H171"
}